{
  "gene_name": "Putative zinc finger protein 702",
  "term_label": "Unknown molecular function",
  "term_id": "UNKNOWN:0001",
  "gene": "UniProtKB:Q9H963",
  "gene_symbol": "ZNF702P"
}